alpha5-beta1 integrin-tissue transglutaminase complex [GO:0071088] (cellular component) Relationships: is a type of plasma membrane protein complex [GO:0098797]; is_a catalytic complex [GO:1902494] Also known as: ITGA5-ITGB1-TGM2 complex Definition: A protein complex that consists of an alpha5-beta1 integrin complex bound to tissue transglutaminase. References: PMID:10684262